glutamine sensor activity [GO:0140786] (molecular function) Definition: Binding to and responding, e.g. by conformational change, to changes in the cellular level of glutamine. Relationships: is_a amino acid sensor activity [GO:0140785] References: PMID:34535752 Also known as: glutamine sensing activity